negative regulation of cell wall organization or biogenesis [GO:1903339] (biological process) Subtypes: negative regulation of secondary cell wall biogenesis [GO:1901347] Also known as: down regulation of cell wall organisation or biogenesis, down regulation of cell wall organization or biogenesis, down regulation of cell wall organization or biogenesis at cellular level, down regulation of cellular cell wall organisation or biogenesis, down regulation of cellular cell wall organization or biogenesis, down-regulation of cell wall organisation or biogenesis, down-regulation of cell wall organization or biogenesis, down-regulation of cell wall organization or biogenesis at cellular level, down-regulation of cellular cell wall organisation or biogenesis, down-regulation of cellular cell wall organization or biogenesis, downregulation of cell wall organisation or biogenesis, downregulation of cell wall organization or biogenesis, downregulation of cell wall organization or biogenesis at cellular level, downregulation of cellular cell wall organisation or biogenesis, downregulation of cellular cell wall organization or biogenesis, negative regulation of cell wall organisation or biogenesis, negative regulation of cell wall organization or biogenesis at cellular level, negative regulation of cellular cell wall organisation or biogenesis, negative regulation of cellular cell wall organization or biogenesis, inhibition of cell wall organisation or biogenesis, inhibition of cell wall organization or biogenesis, inhibition of cell wall organization or biogenesis at cellular level, inhibition of cellular cell wall organisation or biogenesis, inhibition of cellular cell wall organization or biogenesis Relationships: is a type of GO:0048523; is a type of regulation of cell wall organization or biogenesis [GO:1903338]; negatively regulates cell wall organization or biogenesis [GO:0071554] Sources: GOC:TermGenie, GOC:vw, GO_REF:0000058 Definition: Any process that stops, prevents or reduces the frequency, rate or extent of cell wall organization or biogenesis.